{
  "gene": "UniProtKB:P16260",
  "gene_symbol": "SLC25A16",
  "term_label": "coenzyme A transmembrane transporter activity",
  "term_id": "GO:0015228",
  "gene_name": "Solute carrier family 25 member 16"
}